{
  "gene": "UniProtKB:P22792",
  "term_id": "GO:0038023",
  "term_label": "signaling receptor activity",
  "gene_symbol": "CPN2",
  "gene_name": "Carboxypeptidase N subunit 2"
}